{
  "gene_symbol": "ZNF837",
  "term_label": "RNA polymerase II cis-regulatory region sequence-specific DNA binding",
  "gene_name": "Zinc finger protein 837",
  "gene": "UniProtKB:Q96EG3",
  "term_id": "GO:0000978"
}